{
  "gene_name": "Oxysterol-binding protein-related protein 5",
  "gene_symbol": "OSBPL5",
  "gene": "UniProtKB:Q9H0X9",
  "term_label": "cholesterol binding",
  "term_id": "GO:0015485"
}